{
  "gene_name": "Putative olfactory receptor 8G3 pseudogene",
  "term_label": "odorant binding",
  "term_id": "GO:0005549",
  "gene": "UniProtKB:P0DMU2",
  "gene_symbol": "OR8G3"
}